{
  "gene": "UniProtKB:Q64ET8",
  "gene_symbol": "FRG2",
  "term_id": "UNKNOWN:0001",
  "term_label": "Unknown molecular function",
  "gene_name": "Protein FRG2"
}